{
  "term_id": "UNKNOWN:0002",
  "gene_symbol": "SCAND3",
  "gene_name": "SCAN domain-containing protein 3",
  "gene": "UniProtKB:Q6R2W3",
  "term_label": "Unknown biological process"
}